{
  "term_label": "positive regulation of transcription by RNA polymerase II",
  "gene_name": "Heterogeneous nuclear ribonucleoprotein U",
  "gene_symbol": "HNRNPU",
  "gene": "UniProtKB:Q00839",
  "term_id": "GO:0045944"
}